symbiont-induced defense-related programmed cell death [GO:0034050] (biological process) Note: Note that this term is to be used to annotate gene products in the host, not the symbiont. To annotate gene products in the symbiont that induce programmed cell death in the host, consider the biological process term 'symbiont-mediated activation of host programmed cell death' ; GO:0052042'. Definition: Cell death resulting from activation of endogenous cellular processes after interaction with a symbiont (defined as the smaller of two, or more, organisms engaged in symbiosis, a close interaction encompassing mutualism through parasitism). This can be triggered by direct interaction with the organism, for example, contact with penetrating hyphae of a fungus; or an indirect interaction such as symbiont-secreted molecules. Subtypes: plant-type hypersensitive response [GO:0009626] Also known as: host programmed cell death induced by symbiont, programmed cell death induced by symbiont Sources: GOC:pamgo_curators Relationships: is a type of programmed cell death [GO:0012501]; is a type of GO:0140546